{
  "gene_symbol": "ABCC9",
  "gene": "UniProtKB:O60706",
  "gene_name": "ATP-binding cassette sub-family C member 9",
  "term_id": "GO:0140359",
  "term_label": "ABC-type transporter activity"
}